L-propargylglycine--L-glutamate ligase activity [GO:0062145] (molecular function) Definition: Catalysis of the reaction: ATP + L-glutamate + L-propargylglycine = ADP + H+ + L-gamma-glutamyl-L-propargylglycine + phosphate. References: PMID:30867596 Sources: RHEA:59896 Relationships: is a type of GO:0016881